{
  "term_label": "signal transduction",
  "gene": "UniProtKB:Q14002",
  "gene_name": "Carcinoembryonic antigen-related cell adhesion molecule 7",
  "gene_symbol": "CEACAM7",
  "term_id": "GO:0007165"
}